{
  "gene_symbol": "TNXA",
  "term_id": "UNKNOWN:0002",
  "gene": "UniProtKB:Q16473",
  "term_label": "Unknown biological process",
  "gene_name": "Putative tenascin-XA"
}